{
  "gene": "UniProtKB:Q5HYN5",
  "gene_name": "Cancer_testis antigen family 45 member A1",
  "term_label": "Unknown molecular function",
  "gene_symbol": "CT45A1",
  "term_id": "UNKNOWN:0001"
}